regulation of defense response to virus by host [GO:0050691] (biological process) Definition: Any host process that modulates the frequency, rate, or extent of the antiviral response of a host cell or organism. Subtypes: positive regulation of defense response to virus by host [GO:0002230], negative regulation of defense response to virus by host [GO:0050689] Sources: GOC:ai, GOC:dph Also known as: host regulation of antiviral response, regulation by host of antiviral response, regulation of antiviral response by host Relationships: is a type of regulation of defense response to virus [GO:0050688]